{
  "term_id": "GO:0005509",
  "gene_symbol": "CCDC47",
  "gene_name": "PAT complex subunit CCDC47",
  "gene": "UniProtKB:Q96A33",
  "term_label": "calcium ion binding"
}